cellular response to vascular endothelial growth factor stimulus [GO:0035924] (BP) Definition: Any process that results in a change in state or activity of a cell (in terms of movement, secretion, enzyme production, gene expression, etc.) as a result of a vascular endothelial growth factor stimulus. Relationships: is a type of cellular response to growth factor stimulus [GO:0071363] Regulation: regulated by GO:1902547; negatively regulated by negative regulation of cellular response to vascular endothelial growth factor stimulus [GO:1902548] References: PMID:18440775 Sources: GOC:BHF, GOC:rl Also known as: cellular response to VEGF, cellular response to vascular endothelial growth factor, cellular response to VEGFA, cellular response to VEGFB